{
  "term_label": "fumarate transport",
  "term_id": "GO:0015741",
  "gene_name": "Na(+)_citrate cotransporter",
  "gene": "UniProtKB:Q86YT5",
  "gene_symbol": "SLC13A5"
}